{
  "gene_symbol": "YPEL5",
  "term_label": "Unknown biological process",
  "gene": "UniProtKB:P62699",
  "term_id": "UNKNOWN:0002",
  "gene_name": "Protein yippee-like 5"
}